{
  "gene_name": "High mobility group protein B4",
  "gene": "UniProtKB:Q8WW32",
  "term_label": "Unknown molecular function",
  "gene_symbol": "HMGB4",
  "term_id": "UNKNOWN:0001"
}